osteoclast fusion [GO:0072675] (biological process) References: PMID:12713016 Sources: CL:0000092, CL:0000779, GOC:BHF, GOC:mah Definition: The plasma membrane fusion process that results in fusion of mononuclear osteoclasts to form a multinuclear osteoclast. Relationships: is a type of syncytium formation by plasma membrane fusion [GO:0000768]; is part of multinuclear osteoclast differentiation [GO:0072674]